{
  "gene": "UniProtKB:Q96NW7",
  "term_id": "GO:0045211",
  "term_label": "postsynaptic membrane",
  "gene_name": "Leucine-rich repeat-containing protein 7",
  "gene_symbol": "LRRC7"
}